{
  "gene_symbol": "ELOVL2",
  "term_label": "very long-chain fatty acid biosynthetic process",
  "term_id": "GO:0042761",
  "gene": "UniProtKB:Q9NXB9",
  "gene_name": "Elongation of very long chain fatty acids protein 2"
}